{
  "term_label": "cytoplasm",
  "gene_name": "Nucleic acid dioxygenase ALKBH1",
  "gene_symbol": "ALKBH1",
  "term_id": "GO:0005737",
  "gene": "UniProtKB:Q13686"
}